{
  "term_id": "UNKNOWN:0001",
  "term_label": "Unknown molecular function",
  "gene_symbol": "MRPS30",
  "gene": "UniProtKB:Q9NP92",
  "gene_name": "Large ribosomal subunit protein mL65"
}